{
  "gene_name": "E3 ubiquitin-protein ligase pellino homolog 2",
  "gene_symbol": "PELI2",
  "term_id": "GO:0061630",
  "gene": "UniProtKB:Q9HAT8",
  "term_label": "ubiquitin protein ligase activity"
}